{
  "gene_symbol": "OR52I1",
  "term_label": "plasma membrane",
  "gene": "UniProtKB:Q8NGK6",
  "term_id": "GO:0005886",
  "gene_name": "Olfactory receptor 52I1"
}